{
  "gene_name": "Phosphatidylinositol 4,5-bisphosphate 3-kinase catalytic subunit beta isoform",
  "term_id": "GO:0005942",
  "gene_symbol": "PIK3CB",
  "term_label": "phosphatidylinositol 3-kinase complex",
  "gene": "UniProtKB:P42338"
}